{
  "gene_symbol": "FZD7",
  "term_label": "Wnt receptor activity",
  "gene_name": "Frizzled-7",
  "gene": "UniProtKB:O75084",
  "term_id": "GO:0042813"
}